{
  "gene_symbol": "VCPKMT",
  "gene": "UniProtKB:Q9H867",
  "gene_name": "Protein N-lysine methyltransferase METTL21D",
  "term_id": "GO:0005829",
  "term_label": "cytosol"
}